{
  "gene_name": "MHC class I polypeptide-related sequence B",
  "term_label": "immune response",
  "gene": "UniProtKB:Q29980",
  "term_id": "GO:0006955",
  "gene_symbol": "MICB"
}